methanesulfonate monooxygenase activity [GO:0018648] (molecular function) Also known as: methanesulfonate,NADH:oxygen oxidoreductase activity, methanesulphonic acid monooxygenase activity, MSA monooxygenase activity, MSAMO activity, mesylate monooxygenase activity, methanesulfonate,FMNH2:oxygen oxidoreductase activity, methanesulfonic acid monooxygenase activity Definition: Catalysis of the reaction: methanesulfonate + NADH + H+ + O2 = formaldehyde + NAD+ + sulfite + H2O. Sources: EC:1.14.13.111 Relationships: is_a oxidoreductase activity, acting on paired donors, with incorporation or reduction of molecular oxygen, NAD(P)H as one donor, and incorporation of one atom of oxygen [GO:0016709]